{
  "gene_symbol": "IFT43",
  "term_label": "cilium",
  "term_id": "GO:0005929",
  "gene": "UniProtKB:Q96FT9",
  "gene_name": "Intraflagellar transport protein 43 homolog"
}